{
  "term_id": "GO:0004866",
  "term_label": "endopeptidase inhibitor activity",
  "gene_symbol": "AHSG",
  "gene": "UniProtKB:P02765",
  "gene_name": "Alpha-2-HS-glycoprotein"
}